{
  "gene": "UniProtKB:Q5T7P8",
  "gene_symbol": "SYT6",
  "term_id": "GO:0016192",
  "term_label": "vesicle-mediated transport",
  "gene_name": "Synaptotagmin-6"
}